{
  "gene_symbol": "RELB",
  "gene_name": "Transcription factor RelB",
  "gene": "UniProtKB:Q01201",
  "term_label": "DNA-binding transcription factor activity, RNA polymerase II-specific",
  "term_id": "GO:0000981"
}